{
  "gene": "UniProtKB:A6NIR3",
  "gene_symbol": "AGAP5",
  "term_id": "GO:0003924",
  "gene_name": "Arf-GAP with GTPase, ANK repeat and PH domain-containing protein 5",
  "term_label": "GTPase activity"
}